negative regulation of adult somatic muscle development [GO:0062228] (BP) Definition: Any process that decreases the rate, frequency or extent of adult somatic muscle development. Relationships: is a type of GO:0062225; is a type of regulation of adult somatic muscle development [GO:0062226]; RO_0002212 adult somatic muscle development [GO:0007527] References: PMID:16643882, PMID:25758712